{
  "term_id": "GO:0005886",
  "term_label": "plasma membrane",
  "gene_name": "Long-chain fatty acid transport protein 6",
  "gene": "UniProtKB:Q9Y2P4",
  "gene_symbol": "SLC27A6"
}